central region of growth cone [GO:0090724] (cellular component) Relationships: is a type of cellular anatomical structure [GO:0110165]; is part of growth cone [GO:0030426] Definition: The center of the migrating motile tip of a growing nerve cell axon or dendrite. References: PMID:16260607 Sources: GOC:sl